{
  "gene": "UniProtKB:Q9BPW5",
  "gene_symbol": "RASL11B",
  "term_id": "UNKNOWN:0002",
  "term_label": "Unknown biological process",
  "gene_name": "Ras-like protein family member 11B"
}